{
  "gene": "UniProtKB:A8MVW5",
  "term_label": "Golgi apparatus",
  "term_id": "GO:0005794",
  "gene_symbol": "HEPACAM2",
  "gene_name": "HEPACAM family member 2"
}